selenocysteine biosynthetic process [GO:0016260] (biological process) Definition: The chemical reactions and pathways resulting in the formation of selenocysteine, an essential component of glutathione peroxidase and some other proteins. Sources: GOC:go_curators, ISBN:0198506732 Relationships: is a type of GO:0009070; is a type of selenocysteine metabolic process [GO:0016259] Also known as: selenocysteine anabolism, selenocysteine biosynthesis, selenocysteine formation, selenocysteine synthesis